{
  "gene": "UniProtKB:E5RQL4",
  "gene_name": "Formiminotransferase N-terminal subdomain-containing protein",
  "gene_symbol": "FTCDNL1",
  "term_label": "Unknown cellular component",
  "term_id": "UNKNOWN:0003"
}